{
  "term_label": "protein kinase regulator activity",
  "gene_name": "Autophagy-related protein 13",
  "term_id": "GO:0019887",
  "gene": "UniProtKB:O75143",
  "gene_symbol": "ATG13"
}